{
  "term_id": "GO:0005576",
  "gene_symbol": "AHSG",
  "gene_name": "Alpha-2-HS-glycoprotein",
  "term_label": "extracellular region",
  "gene": "UniProtKB:P02765"
}